collecting lymphatic vessel constriction [GO:1990192] (biological process) Definition: A decrease in the diameter of collecting lymphatic vessels. Also known as: lymphatic vessel myogenic constriction References: PMID:23322290 Regulation: regulated by regulation of collecting lymphatic vessel constriction [GO:1903814]; negatively regulated by GO:1903815; positively regulated by GO:1903816 Relationships: is a type of regulation of lymphatic vessel size [GO:1990186]